host defense response against symbiont-mediated perturbation of plasma membrane integrity [GO:0140976] (BP) Also known as: defense response against disruption of plasma membrane integrity, defense response against perturbation of plasma membrane integrity References: PMID:17234446, PMID:21518219 Definition: The cellular processes and signaling pathways by which a cell responds to disruption of the integrity of its plasma membrane by another organism. Some toxins produced by other organisms can form pores in membranes, or affect the membrane permeability. Relationships: is a type of defense response to symbiont [GO:0140546]